{
  "gene_symbol": "BARX1",
  "term_label": "DNA-binding transcription factor activity, RNA polymerase II-specific",
  "gene": "UniProtKB:Q9HBU1",
  "term_id": "GO:0000981",
  "gene_name": "Homeobox protein BarH-like 1"
}